zymogen granule membrane [GO:0042589] (cellular component) Sources: GOC:jl Relationships: is a type of GO:0030667; BFO_0000050 zymogen granule [GO:0042588] Definition: The lipid bilayer surrounding a zymogen granule.